T cell aggregation [GO:0070489] (biological process) Definition: The adhesion of one T cell to one or more other T cells via adhesion molecules. Subtypes: thymocyte aggregation [GO:0071594] Also known as: T lymphocyte aggregation, T-cell aggregation, T-lymphocyte aggregation Relationships: is a type of GO:0071593 References: PMID:12972508 Sources: GOC:sl